regulation of G1 to G0 transition [GO:1903450] (biological process) Relationships: is a type of regulation of cell cycle process [GO:0010564]; regulates G1 to G0 transition [GO:0070314] References: PMID:24088570 Sources: GOC:TermGenie, GOC:di, GO_REF:0000058 Also known as: regulation of G1/G0 transition, regulation of establishment of cell quiescence, regulation of cell cycle quiescence, regulation of stationary phase Definition: Any process that modulates the frequency, rate or extent of G1 to G0 transition. Subtypes: negative regulation of G1 to G0 transition [GO:1903451], GO:1903452